{
  "term_id": "GO:0030154",
  "gene": "UniProtKB:P10826",
  "term_label": "cell differentiation",
  "gene_symbol": "RARB",
  "gene_name": "Retinoic acid receptor beta"
}